{
  "gene": "UniProtKB:O60733",
  "gene_symbol": "PLA2G6",
  "gene_name": "85_88 kDa calcium-independent phospholipase A2",
  "term_id": "GO:0047499",
  "term_label": "calcium-independent phospholipase A2 activity"
}